{
  "gene": "UniProtKB:Q96HD9",
  "gene_name": "N-acyl-aromatic-L-amino acid amidohydrolase (carboxylate-forming)",
  "gene_symbol": "ACY3",
  "term_label": "Unknown biological process",
  "term_id": "UNKNOWN:0002"
}